{
  "term_id": "UNKNOWN:0002",
  "gene": "UniProtKB:Q8IYK8",
  "gene_name": "GTP-binding protein REM 2",
  "term_label": "Unknown biological process",
  "gene_symbol": "REM2"
}